{
  "gene_symbol": "ZNF750",
  "gene_name": "Zinc finger protein 750",
  "term_label": "epidermis development",
  "term_id": "GO:0008544",
  "gene": "UniProtKB:Q32MQ0"
}